2-chloro-4-hydroxy-6-amino-1,3,5-triazine aminohydrolase activity [GO:0018755] (molecular function) Sources: UM-BBD_reactionID:r1414 Definition: Catalysis of the reaction: 2-chloro-4-hydroxy-6-amino-1,3,5-triazine + OH- = 2,4-dihydroxy-6-amino-1,3,5-triazine + Cl-. Relationships: is a type of hydrolase activity, acting on carbon-nitrogen (but not peptide) bonds, in linear amidines [GO:0016813]